spermidine:feruloyl CoA N-acyltransferase activity [GO:0080075] (molecular function) Relationships: is a type of N-acyltransferase activity [GO:0016410] References: PMID:19077165 Definition: Catalysis of the transfer of a feruloyl group to a nitrogen atom on the spermidine molecule.